{
  "term_id": "GO:1990431",
  "gene_name": "Poly(A)-specific ribonuclease PARN",
  "gene_symbol": "PARN",
  "term_label": "priRNA 3'-end processing",
  "gene": "UniProtKB:O95453"
}